{
  "gene_name": "Methyltransferase-like protein 22",
  "term_label": "Unknown biological process",
  "term_id": "UNKNOWN:0002",
  "gene_symbol": "METTL22",
  "gene": "UniProtKB:Q9BUU2"
}